mitotic nuclear membrane biogenesis [GO:0101026] (biological process) Definition: A process in which the nuclear inner or outer membrane is synthesized, aggregates, and bonds together during mitotic nuclear division. Also known as: nuclear membrane biogenesis involved in mitotic nuclear division References: PMID:26869222 Sources: GOC:vw Relationships: is a type of membrane organization [GO:0061024]; is a type of nuclear membrane biogenesis [GO:0101025]; is_a GO:1903047; is part of mitotic nuclear division [GO:0140014]